structural constituent of tooth enamel [GO:0030345] (molecular function) Sources: GOC:mah Relationships: is a type of extracellular matrix structural constituent conferring compression resistance [GO:0030021] Definition: The action of a molecule that contributes to the structural integrity of tooth enamel.